neuropeptide processing [GO:0061837] (biological process) Relationships: is a type of signaling receptor ligand precursor processing [GO:0140448] Definition: Any protein maturation process achieved by the cleavage of a peptide bond or bonds within a neuropeptide precursor. Processing leads to the attainment of the full functional capacity of the neuropeptide. References: PMID:12657671, PMID:17564681